{
  "gene_symbol": "BMP2KL",
  "term_label": "Unknown cellular component",
  "term_id": "UNKNOWN:0003",
  "gene": "UniProtKB:Q5H9B9",
  "gene_name": "Putative BMP-2-inducible kinase-like protein"
}